{
  "gene": "UniProtKB:Q8TE60",
  "gene_symbol": "ADAMTS18",
  "term_label": "extracellular matrix",
  "gene_name": "A disintegrin and metalloproteinase with thrombospondin motifs 18",
  "term_id": "GO:0031012"
}